{
  "gene_symbol": "SLC27A4",
  "term_id": "GO:0090434",
  "term_label": "oleoyl-CoA ligase activity",
  "gene": "UniProtKB:Q6P1M0",
  "gene_name": "Long-chain fatty acid transport protein 4"
}